oxidoreductase activity, acting on paired donors, with incorporation or reduction of molecular oxygen, with 2-oxoglutarate as one donor, and the other dehydrogenated [GO:0050498] (molecular function) Definition: Catalysis of an oxidation-reduction (redox) reaction in which hydrogen or electrons are transferred from 2-oxoglutarate and one other donor, and the latter donor is dehydrogenated. Subtypes: GO:0050599, L-lysine 4-chlorinase activity [GO:0062147], GO:0102717 Sources: EC:1.14.20.- Relationships: is_a oxidoreductase activity, acting on paired donors, with incorporation or reduction of molecular oxygen [GO:0016705]